{
  "gene_symbol": "TRIM56",
  "gene_name": "E3 ubiquitin-protein ligase TRIM56",
  "term_label": "ubiquitin protein ligase activity",
  "term_id": "GO:0061630",
  "gene": "UniProtKB:Q9BRZ2"
}